{
  "gene_name": "Translocating chain-associated membrane protein 2",
  "gene_symbol": "TRAM2",
  "term_id": "GO:0045048",
  "gene": "UniProtKB:Q15035",
  "term_label": "protein insertion into ER membrane"
}